{
  "gene": "UniProtKB:Q96MI6",
  "term_id": "GO:0004741",
  "gene_symbol": "PPM1M",
  "term_label": "[pyruvate dehydrogenase (acetyl-transferring)]-phosphatase activity",
  "gene_name": "Protein phosphatase 1M"
}